{
  "gene": "UniProtKB:Q8WX39",
  "gene_name": "Epididymal-specific lipocalin-9",
  "gene_symbol": "LCN9",
  "term_id": "GO:0005615",
  "term_label": "extracellular space"
}